{
  "term_id": "GO:0001227",
  "term_label": "DNA-binding transcription repressor activity, RNA polymerase II-specific",
  "gene_symbol": "HIC2",
  "gene": "UniProtKB:Q96JB3",
  "gene_name": "Hypermethylated in cancer 2 protein"
}